omega-3 fatty acid desaturase activity [GO:0042389] (molecular function) Definition: Catalysis of the introduction of an omega-3 double bond into the fatty acid hydrocarbon chain. References: PMID:9037020 Sources: GOC:jl Relationships: is a type of oxidoreductase activity, acting on paired donors, with incorporation or reduction of molecular oxygen [GO:0016705]